4-(2-carboxyphenyl)-2-oxobut-3-enoate aldolase activity [GO:0018803] (molecular function) Definition: Catalysis of the reaction: (3E)-4-(2-carboxyphenyl)-2-oxobut-3-enoate = 2-carboxybenzaldehyde + pyruvate. Also known as: trans-2'-carboxybenzalpyruvate hydratase-aldolase activity, (3E)-4-(2-carboxyphenyl)-2-oxobut-3-enoate 2-carboxybenzaldehyde-lyase activity, (3Z)-4-(2-carboxyphenyl)-2-oxobut-3-enoate 2-carboxybenzaldehyde-lyase activity, (3Z)-4-(2-carboxyphenyl)-2-oxobut-3-enoate 2-carboxybenzaldehyde-lyase (pyruvate-forming), 2'-carboxybenzalpyruvate aldolase activity Sources: EC:4.1.2.34 Relationships: is a type of carboxy-lyase activity [GO:0016831]